cell-cell adhesion involved in neuronal-glial interactions involved in cerebral cortex radial glia guided migration [GO:0021813] (biological process) Definition: The interaction between two cells that modulates the association of a neuronal cell and a glial cell involved in glial-mediated radial cell migration in the cerebral cortex. References: PMID:12626695 Sources: GOC:cls, GOC:dgh, GOC:dph, GOC:jid, GO_REF:0000021 Also known as: cell-cell adhesion involved in neuronal-glial interactions involved in cerebral cortex glial-mediated radial migration Relationships: is a type of cell-cell adhesion [GO:0098609]; is part of neuronal-glial interaction involved in cerebral cortex radial glia guided migration [GO:0021812]